{
  "gene_symbol": "OPTC",
  "term_id": "GO:0060348",
  "gene": "UniProtKB:Q9UBM4",
  "term_label": "bone development",
  "gene_name": "Opticin"
}